{
  "term_label": "Unknown molecular function",
  "gene_symbol": "IDH3G",
  "gene_name": "Isocitrate dehydrogenase [NAD] subunit gamma, mitochondrial",
  "gene": "UniProtKB:P51553",
  "term_id": "UNKNOWN:0001"
}